{
  "gene_symbol": "BRS3",
  "term_id": "GO:0005886",
  "gene": "UniProtKB:P32247",
  "term_label": "plasma membrane",
  "gene_name": "Bombesin receptor subtype-3"
}